intestinal absorption [GO:0050892] (biological process) Definition: A process in which nutrients are taken up from the contents of the intestine. Sources: GOC:ai, GOC:dph Relationships: is_a digestive system process [GO:0022600] Subtypes: intestinal folate absorption [GO:0098829], intestinal lipid absorption [GO:0098856], GO:0106001, intestinal iron absorption [GO:0160179] Regulation: regulated by regulation of intestinal absorption [GO:1904478]; RO_0002212 by negative regulation of intestinal absorption [GO:1904479]; positively regulated by positive regulation of intestinal absorption [GO:1904480]